{
  "term_label": "membrane",
  "gene": "UniProtKB:P98153",
  "gene_symbol": "DGCR2",
  "gene_name": "Integral membrane protein DGCR2_IDD",
  "term_id": "GO:0016020"
}